{
  "gene_name": "Septin-2",
  "gene": "UniProtKB:Q15019",
  "term_label": "molecular adaptor activity",
  "term_id": "GO:0060090",
  "gene_symbol": "SEPTIN2"
}